{
  "term_id": "GO:0016922",
  "gene_name": "Nuclear receptor coactivator 3",
  "gene": "UniProtKB:Q9Y6Q9",
  "term_label": "nuclear receptor binding",
  "gene_symbol": "NCOA3"
}